{
  "gene_name": "Protocadherin beta-2",
  "term_label": "cell adhesion molecule binding",
  "gene_symbol": "PCDHB2",
  "gene": "UniProtKB:Q9Y5E7",
  "term_id": "GO:0050839"
}